{
  "gene_symbol": "MTFR2",
  "gene_name": "Mitochondrial fission regulator 2",
  "term_label": "mitochondrion",
  "gene": "UniProtKB:Q6P444",
  "term_id": "GO:0005739"
}